{
  "term_label": "cerebral cortex development",
  "term_id": "GO:0021987",
  "gene_symbol": "TACC3",
  "gene_name": "Transforming acidic coiled-coil-containing protein 3",
  "gene": "UniProtKB:Q9Y6A5"
}